{
  "term_label": "Unknown molecular function",
  "gene": "UniProtKB:O60290",
  "gene_symbol": "ZNF862",
  "term_id": "UNKNOWN:0001",
  "gene_name": "Zinc finger protein 862"
}